peptidyl-threonine modification [GO:0018210] (BP) Definition: The modification of peptidyl-threonine. Subtypes: peptidyl-threonine phosphorylation [GO:0018107], peptidyl-threonine O-acetylation [GO:0120258] Relationships: is a type of GO:0018193 Sources: GOC:go_curators